{
  "gene": "UniProtKB:P61218",
  "term_id": "GO:0042797",
  "gene_symbol": "POLR2F",
  "gene_name": "DNA-directed RNA polymerases I, II, and III subunit RPABC2",
  "term_label": "tRNA transcription by RNA polymerase III"
}